{
  "gene": "UniProtKB:Q96QA6",
  "gene_name": "Protein yippee-like 2",
  "gene_symbol": "YPEL2",
  "term_label": "Unknown biological process",
  "term_id": "UNKNOWN:0002"
}